{
  "gene_name": "Glutamate receptor 2",
  "term_label": "postsynaptic density membrane",
  "term_id": "GO:0098839",
  "gene_symbol": "GRIA2",
  "gene": "UniProtKB:P42262"
}